{
  "gene": "UniProtKB:Q8NFY9",
  "gene_symbol": "KBTBD8",
  "term_label": "cytoplasm",
  "gene_name": "Kelch repeat and BTB domain-containing protein 8",
  "term_id": "GO:0005737"
}